{
  "gene_symbol": "YAP1",
  "gene": "UniProtKB:P46937",
  "term_label": "positive regulation of epithelial cell proliferation",
  "term_id": "GO:0050679",
  "gene_name": "Transcriptional coactivator YAP1"
}